{
  "gene": "UniProtKB:P49326",
  "term_label": "Unknown cellular component",
  "gene_symbol": "FMO5",
  "gene_name": "Flavin-containing monooxygenase 5",
  "term_id": "UNKNOWN:0003"
}